{
  "term_label": "Unknown molecular function",
  "gene_symbol": "TMEM169",
  "gene_name": "Transmembrane protein 169",
  "gene": "UniProtKB:Q96HH4",
  "term_id": "UNKNOWN:0001"
}